{
  "gene_symbol": "CBX6",
  "gene_name": "Chromobox protein homolog 6",
  "gene": "UniProtKB:O95503",
  "term_id": "GO:0003682",
  "term_label": "chromatin binding"
}